{
  "gene": "UniProtKB:Q9C0K3",
  "gene_symbol": "ACTR3C",
  "term_id": "UNKNOWN:0003",
  "term_label": "Unknown cellular component",
  "gene_name": "Actin-related protein 3C"
}